{
  "term_label": "positive regulation of protein targeting to membrane",
  "term_id": "GO:0090314",
  "gene": "UniProtKB:A6NFQ2",
  "gene_name": "TRPM8 channel-associated factor 2",
  "gene_symbol": "TCAF2"
}